{
  "term_label": "Unknown biological process",
  "gene_symbol": "SLFNL1",
  "gene": "UniProtKB:Q499Z3",
  "gene_name": "Schlafen-like protein 1",
  "term_id": "UNKNOWN:0002"
}